{
  "gene_name": "Beta-defensin 114",
  "term_label": "extracellular space",
  "gene": "UniProtKB:Q30KQ6",
  "gene_symbol": "DEFB114",
  "term_id": "GO:0005615"
}